{
  "gene": "UniProtKB:Q15058",
  "term_label": "microtubule binding",
  "gene_name": "Kinesin-like protein KIF14",
  "gene_symbol": "KIF14",
  "term_id": "GO:0008017"
}